negative regulation of translational initiation by iron [GO:0045993] (biological process) Also known as: down regulation of translational initiation by iron, down-regulation of translational initiation by iron, downregulation of translational initiation by iron, inhibition of translational initiation by iron Definition: Any process involving iron that stops, prevents or reduces the rate of translational initiation. Relationships: is a type of regulation of translational initiation by iron [GO:0006447]; is a type of negative regulation of translational initiation [GO:0045947] Sources: GOC:go_curators